regulation of hemopoiesis [GO:1903706] (biological process) References: PMID:20080761 Sources: GOC:PARL, GOC:TermGenie, GOC:pad, GO_REF:0000058 Relationships: is a type of regulation of immune system process [GO:0002682]; is a type of regulation of cell development [GO:0060284]; is a type of regulation of multicellular organismal development [GO:2000026]; regulates hemopoiesis [GO:0030097] Note: An example of this is Atg7 in mouse (UniProt symbol, Q9D906) in PMID:20080761, inferred from mutant phenotype. Definition: Any process that modulates the frequency, rate or extent of hemopoiesis. Also known as: regulation of blood cell biosynthesis, regulation of blood cell formation, regulation of haemopoiesis, regulation of hematopoiesis Subtypes: GO:0035203, regulation of myeloid cell differentiation [GO:0045637], regulation of leukocyte differentiation [GO:1902105], negative regulation of hemopoiesis [GO:1903707], positive regulation of hemopoiesis [GO:1903708], regulation of osteoclast development [GO:2001204]